{
  "gene": "UniProtKB:Q6DN03",
  "term_id": "GO:0006325",
  "gene_name": "Putative histone H2B type 2-C",
  "term_label": "chromatin organization",
  "gene_symbol": "H2BC20P"
}